interleukin-11 receptor activity [GO:0004921] (molecular function) Definition: Combining with interleukin-11 and transmitting the signal from one side of the membrane to the other to initiate a change in cell activity. Sources: GOC:jl, GOC:signaling Relationships: is a type of GO:0004896; is part of GO:0038154; has part interleukin-11 binding [GO:0019970] Also known as: IL-11 receptor activity, IL-11R, gp130